{
  "term_id": "GO:0070402",
  "gene_name": "Quinone oxidoreductase",
  "gene_symbol": "CRYZ",
  "term_label": "NADPH binding",
  "gene": "UniProtKB:Q08257"
}